{
  "gene_symbol": "PRKRA",
  "gene": "UniProtKB:O75569",
  "term_id": "GO:0016442",
  "term_label": "RISC complex",
  "gene_name": "Interferon-inducible double-stranded RNA-dependent protein kinase activator A"
}